{
  "gene_name": "F-box_LRR-repeat protein 16",
  "term_id": "GO:0031146",
  "term_label": "SCF-dependent proteasomal ubiquitin-dependent protein catabolic process",
  "gene_symbol": "FBXL16",
  "gene": "UniProtKB:Q8N461"
}